{
  "gene_symbol": "EFCAB11",
  "term_id": "GO:0005737",
  "gene": "UniProtKB:Q9BUY7",
  "gene_name": "EF-hand calcium-binding domain-containing protein 11",
  "term_label": "cytoplasm"
}